{
  "term_label": "heme binding",
  "gene": "UniProtKB:Q6VVX0",
  "gene_name": "Vitamin D 25-hydroxylase",
  "term_id": "GO:0020037",
  "gene_symbol": "CYP2R1"
}